GGC codon-amino acid adaptor activity [GO:0033462] (molecular function) Also known as: glycine tRNA Sources: GOC:mah Note: Note that in the standard genetic code, GGC codes for glycine. Relationships: is a type of triplet codon-amino acid adaptor activity [GO:0030533] Definition: A triplet codon-amino acid adaptor activity that recognizes a GGC codon.